{
  "gene_name": "Protein 4.1",
  "gene_symbol": "EPB41",
  "gene": "UniProtKB:P11171",
  "term_label": "actomyosin structure organization",
  "term_id": "GO:0031032"
}